{
  "gene_name": "Sodium- and chloride-dependent neutral and basic amino acid transporter B(0+)",
  "gene": "UniProtKB:Q9UN76",
  "term_id": "GO:0015657",
  "gene_symbol": "SLC6A14",
  "term_label": "branched-chain amino acid:sodium symporter activity"
}